{
  "gene_symbol": "MBNL2",
  "term_label": "RNA binding",
  "gene": "UniProtKB:Q5VZF2",
  "gene_name": "Muscleblind-like protein 2",
  "term_id": "GO:0003723"
}